{
  "term_label": "negative regulation of transcription by RNA polymerase II",
  "gene": "UniProtKB:A8MXT2",
  "gene_symbol": "MAGEB17",
  "gene_name": "Melanoma-associated antigen B17",
  "term_id": "GO:0000122"
}